{
  "term_id": "GO:0005102",
  "term_label": "signaling receptor binding",
  "gene": "UniProtKB:P14210",
  "gene_name": "Hepatocyte growth factor",
  "gene_symbol": "HGF"
}